{
  "term_label": "Unknown molecular function",
  "gene_name": "Signal peptidase complex subunit 2",
  "term_id": "UNKNOWN:0001",
  "gene": "UniProtKB:Q15005",
  "gene_symbol": "SPCS2"
}